positive regulation of endocrocin biosynthetic process [GO:1900669] (biological process) Relationships: is a type of positive regulation of small molecule metabolic process [GO:0062013]; is_a positive regulation of secondary metabolite biosynthetic process [GO:1900378]; is a type of regulation of endocrocin biosynthetic process [GO:1900667]; positively regulates endocrocin biosynthetic process [GO:1900602] Definition: Any process that activates or increases the frequency, rate or extent of endocrocin biosynthetic process. Sources: GOC:TermGenie, GOC:di Also known as: activation of endocrocin anabolism, activation of endocrocin biosynthesis, activation of endocrocin formation, activation of endocrocin synthesis, positive regulation of endocrocin anabolism, positive regulation of endocrocin biosynthesis, positive regulation of endocrocin formation, positive regulation of endocrocin synthesis, up regulation of endocrocin anabolism, up regulation of endocrocin biosynthesis, up regulation of endocrocin biosynthetic process, up regulation of endocrocin formation, up regulation of endocrocin synthesis, up-regulation of endocrocin anabolism, up-regulation of endocrocin biosynthesis, up-regulation of endocrocin biosynthetic process, up-regulation of endocrocin formation, up-regulation of endocrocin synthesis, upregulation of endocrocin anabolism, upregulation of endocrocin biosynthesis, upregulation of endocrocin biosynthetic process, upregulation of endocrocin formation, upregulation of endocrocin synthesis, activation of endocrocin biosynthetic process